{
  "gene": "UniProtKB:Q9NPC1",
  "term_label": "plasma membrane",
  "term_id": "GO:0005886",
  "gene_symbol": "LTB4R2",
  "gene_name": "Leukotriene B4 receptor 2"
}